{
  "gene_name": "Nucleolar protein 3",
  "gene_symbol": "NOL3",
  "gene": "UniProtKB:O60936",
  "term_label": "cysteine-type endopeptidase inhibitor activity involved in apoptotic process",
  "term_id": "GO:0043027"
}